{
  "term_id": "GO:0048666",
  "term_label": "neuron development",
  "gene_symbol": "DRGX",
  "gene_name": "Dorsal root ganglia homeobox protein",
  "gene": "UniProtKB:A6NNA5"
}